{
  "gene_symbol": "ZNF417",
  "gene": "UniProtKB:Q8TAU3",
  "gene_name": "Zinc finger protein 417",
  "term_id": "GO:0000981",
  "term_label": "DNA-binding transcription factor activity, RNA polymerase II-specific"
}